{
  "gene_name": "Rab GTPase-activating protein 1",
  "term_label": "GTPase activator activity",
  "gene": "UniProtKB:Q9Y3P9",
  "term_id": "GO:0005096",
  "gene_symbol": "RABGAP1"
}